{
  "gene_name": "Fatty acid CoA ligase Acsl3",
  "gene": "UniProtKB:O95573",
  "gene_symbol": "ACSL3",
  "term_label": "plasma membrane",
  "term_id": "GO:0005886"
}